{
  "term_label": "Unknown cellular component",
  "term_id": "UNKNOWN:0003",
  "gene_symbol": "ERICH3",
  "gene": "UniProtKB:Q5RHP9",
  "gene_name": "Glutamate-rich protein 3"
}